{
  "gene_name": "Zinc finger protein with KRAB and SCAN domains 7",
  "gene_symbol": "ZKSCAN7",
  "gene": "UniProtKB:Q9P0L1",
  "term_label": "RNA polymerase II cis-regulatory region sequence-specific DNA binding",
  "term_id": "GO:0000978"
}